tartrate decarboxylase activity [GO:0050319] (molecular function) Relationships: is a type of carboxy-lyase activity [GO:0016831] Definition: Catalysis of the reaction: L-tartrate + H+ = D-glycerate + CO2. Sources: EC:4.1.1.73, RHEA:13317 Also known as: (R,R)-tartrate carboxy-lyase (D-glycerate-forming), (R,R)-tartrate carboxy-lyase activity